pyocyanine biosynthetic process [GO:0106220] (biological process) Also known as: pyocyanin biosynthetic process Relationships: is a type of GO:0009058 Regulation: RO_0002211 by regulation of pyocyanine biosynthetic process [GO:0062161]; positively regulated by positive regulation of pyocyanine biosynthetic process [GO:0062162] Definition: The chemical reactions and pathways resulting in the formation of pyrocyanin, an iminium betaine that is 5-methylphenazin-5-ium which is substituted at position 1 by an oxidanidyl group. References: PMID:28715477